{
  "gene_symbol": "RAB14",
  "term_label": "phagolysosome assembly",
  "gene_name": "Ras-related protein Rab-14",
  "term_id": "GO:0001845",
  "gene": "UniProtKB:P61106"
}